{
  "gene_symbol": "CDK13",
  "term_label": "positive regulation of transcription elongation by RNA polymerase II",
  "gene_name": "Cyclin-dependent kinase 13",
  "term_id": "GO:0032968",
  "gene": "UniProtKB:Q14004"
}